{
  "term_id": "UNKNOWN:0002",
  "gene_symbol": "VWA8",
  "term_label": "Unknown biological process",
  "gene": "UniProtKB:A3KMH1",
  "gene_name": "von Willebrand factor A domain-containing protein 8"
}